{
  "term_label": "desensitization of G protein-coupled receptor signaling pathway",
  "gene_name": "Lymphocyte antigen 6 family member G6E",
  "term_id": "GO:0002029",
  "gene_symbol": "LY6G6E",
  "gene": "UniProtKB:A0A0B4J1T7"
}